{
  "gene": "UniProtKB:Q9BXI3",
  "term_id": "GO:0005829",
  "term_label": "cytosol",
  "gene_symbol": "NT5C1A",
  "gene_name": "Cytosolic 5'-nucleotidase 1A"
}